{
  "term_label": "ketone body metabolic process",
  "gene_name": "Succinyl-CoA:3-ketoacid coenzyme A transferase 2, mitochondrial",
  "term_id": "GO:1902224",
  "gene": "UniProtKB:Q9BYC2",
  "gene_symbol": "OXCT2"
}